{
  "gene_symbol": "KL",
  "gene_name": "Klotho",
  "gene": "UniProtKB:Q9UEF7",
  "term_id": "GO:0008543",
  "term_label": "fibroblast growth factor receptor signaling pathway"
}